{
  "gene_name": "D(1A) dopamine receptor",
  "term_id": "GO:0001588",
  "gene_symbol": "DRD1",
  "term_label": "dopamine neurotransmitter receptor activity, coupled via Gs",
  "gene": "UniProtKB:P21728"
}